type I transforming growth factor beta receptor binding [GO:0034713] (molecular function) Also known as: TGF-beta type I binding, transforming growth factor beta receptor type I binding, type I TGF-beta binding, babo binding, babo ligand, baboon binding, baboon ligand, baboon receptor ligand, sax binding, sax ligand, saxophone binding, saxophone ligand, thickveins binding, thickveins ligand, tkv binding, tkv ligand, transforming growth factor beta ligand binding to type I receptor Definition: Binding to a type I transforming growth factor beta receptor. Relationships: is a type of transforming growth factor beta receptor binding [GO:0005160] Sources: GOC:BHF, GOC:mah